{
  "gene_symbol": "ASPRV1",
  "gene": "UniProtKB:Q53RT3",
  "term_id": "UNKNOWN:0002",
  "gene_name": "Retroviral-like aspartic protease 1",
  "term_label": "Unknown biological process"
}